{
  "gene": "UniProtKB:O43663",
  "gene_symbol": "PRC1",
  "gene_name": "Protein regulator of cytokinesis 1",
  "term_id": "GO:0051256",
  "term_label": "mitotic spindle midzone assembly"
}